clathrin-coated phagocytic vesicle membrane [GO:0030671] (cellular component) Relationships: is a type of clathrin-coated endocytic vesicle membrane [GO:0030669]; is a type of phagocytic vesicle membrane [GO:0030670]; is part of clathrin-coated phagocytic vesicle [GO:0045336] Sources: GOC:mah Definition: The lipid bilayer surrounding a clathrin-coated phagocytic vesicle.